{
  "gene": "UniProtKB:P35414",
  "term_label": "G protein-coupled receptor signaling pathway",
  "gene_name": "Apelin receptor",
  "gene_symbol": "APLNR",
  "term_id": "GO:0007186"
}